inulin biosynthetic process [GO:1902928] (BP) Definition: The chemical reactions and pathways resulting in the formation of inulin. Note: SUC2 in S. cerevisiae strain JZ1C in PMID:23104410. References: PMID:23104410 Sources: GOC:TermGenie, GO_REF:0000068 Also known as: inulin anabolism, inulin biosynthesis, inulin formation, inulin synthesis Relationships: is_a GO:0010146